{
  "gene_symbol": "MAST3",
  "term_label": "protein serine/threonine kinase activity",
  "gene": "UniProtKB:O60307",
  "term_id": "GO:0004674",
  "gene_name": "Microtubule-associated serine_threonine-protein kinase 3"
}